oxalic acid secretion [GO:0046724] (biological process) Also known as: oxalate secretion Relationships: is a type of GO:0019532; is a type of GO:0046717 Definition: The controlled release of oxalic acid, ethanedioic acid, by a cell or a tissue. Sources: GOC:ai